nucleotide-excision repair factor 2 complex [GO:0000111] (cellular component) References: PMID:10915862 Definition: One of several protein complexes involved in nucleotide-excision repair; possesses damaged DNA binding activity. In S. cerevisiae, it is composed of Rad4p and Rad23p. Relationships: is a type of nucleotide-excision repair complex [GO:0000109] Also known as: NEF2 complex Note: Note that process and function information are included in the term and definition for the purpose of describing and distinguishing the complex.